{
  "term_label": "Unknown molecular function",
  "term_id": "UNKNOWN:0001",
  "gene": "UniProtKB:Q5T754",
  "gene_symbol": "LCE1F",
  "gene_name": "Late cornified envelope protein 1F"
}